{
  "term_label": "regulation of gene expression",
  "gene": "UniProtKB:Q9P2D1",
  "term_id": "GO:0010468",
  "gene_symbol": "CHD7",
  "gene_name": "Chromodomain-helicase-DNA-binding protein 7"
}